{
  "gene_symbol": "SCYGR9",
  "term_id": "UNKNOWN:0003",
  "term_label": "Unknown cellular component",
  "gene": "UniProtKB:P0DSO2",
  "gene_name": "Small cysteine and glycine repeat-containing protein 9"
}